{
  "term_id": "GO:0000139",
  "term_label": "Golgi membrane",
  "gene_name": "Galactosylgalactosylxylosylprotein 3-beta-glucuronosyltransferase 3",
  "gene_symbol": "B3GAT3",
  "gene": "UniProtKB:O94766"
}